succinate-semialdehyde dehydrogenase [NAD(P)+] activity [GO:0009013] (molecular function) Definition: Catalysis of the reaction: succinate semialdehyde + NAD(P)+ + H2O = succinate + NAD(P)H + H+. Sources: EC:1.2.1.16 Also known as: succinate semialdehyde dehydrogenase (nicotinamide adenine dinucleotide (phosphate)), succinate-semialdehyde:NAD(P)+ oxidoreductase activity Relationships: is a type of oxidoreductase activity, acting on the aldehyde or oxo group of donors, NAD or NADP as acceptor [GO:0016620] Subtypes: GO:0004777, GO:0036243